{
  "gene_name": "Olfactory receptor 5M3",
  "gene": "UniProtKB:Q8NGP4",
  "gene_symbol": "OR5M3",
  "term_label": "Unknown cellular component",
  "term_id": "UNKNOWN:0003"
}